{
  "term_label": "Unknown biological process",
  "gene_symbol": "KRTAP19-7",
  "gene": "UniProtKB:Q3SYF9",
  "gene_name": "Keratin-associated protein 19-7",
  "term_id": "UNKNOWN:0002"
}